{
  "gene_name": "Regulator of microtubule dynamics protein 2",
  "gene": "UniProtKB:Q96LZ7",
  "term_id": "GO:0005739",
  "gene_symbol": "RMDN2",
  "term_label": "mitochondrion"
}